regulation of neuron projection development [GO:0010975] (biological process) Subtypes: positive regulation of neuron projection development [GO:0010976], negative regulation of neuron projection development [GO:0010977], GO:0050770, regulation of dendrite development [GO:0050773], regulation of dendritic spine morphogenesis [GO:0061001], regulation of neuron projection regeneration [GO:0070570], regulation of axon guidance [GO:1902667] Also known as: regulation of neurite biosynthesis, regulation of neurite development, regulation of neurite formation, regulation of neurite growth Definition: Any process that modulates the rate, frequency or extent of neuron projection development. Neuron projection development is the process whose specific outcome is the progression of a neuron projection over time, from its formation to the mature structure. A neuron projection is any process extending from a neural cell, such as axons or dendrites (collectively called neurites). Sources: GOC:dph, GOC:tb Relationships: is a type of regulation of plasma membrane bounded cell projection organization [GO:0120035]; regulates neuron projection development [GO:0031175]